{
  "term_label": "glutamine transport",
  "gene_name": "Probable sodium-coupled neutral amino acid transporter 6",
  "gene": "UniProtKB:Q8IZM9",
  "term_id": "GO:0006868",
  "gene_symbol": "SLC38A6"
}